{
  "gene_name": "RB1-inducible coiled-coil protein 1",
  "gene": "UniProtKB:Q8TDY2",
  "term_label": "autophagy of mitochondrion",
  "gene_symbol": "RB1CC1",
  "term_id": "GO:0000422"
}